D-glucuronate transmembrane transporter activity [GO:0042880] (molecular function) Relationships: is a type of glucuronate transmembrane transporter activity [GO:0015135]; is part of D-glucuronate transmembrane transport [GO:0042874] Definition: Enables the transfer of D-glucuronate, the D-enantiomer of glucuronate, from one side of a membrane to the other. Sources: GOC:jl, GOC:jsg, GOC:mah, GOC:mtg_transport, ISBN:0198506732